{
  "gene_symbol": "TUBB3",
  "term_label": "microtubule",
  "term_id": "GO:0005874",
  "gene": "UniProtKB:Q13509",
  "gene_name": "Tubulin beta-3 chain"
}